regulation of membrane hyperpolarization [GO:1902630] (biological process) Definition: Any process that modulates the frequency, rate or extent of membrane hyperpolarization. Subtypes: negative regulation of membrane hyperpolarization [GO:1902631], positive regulation of membrane hyperpolarization [GO:1902632] References: PMID:23223304 Sources: GOC:TermGenie, GO_REF:0000058 Relationships: is a type of GO:0042391; is a type of regulation of biological process [GO:0050789]; regulates membrane hyperpolarization [GO:0060081]